{
  "gene_name": "Homeobox protein ARX",
  "term_id": "GO:0005634",
  "term_label": "nucleus",
  "gene": "UniProtKB:Q96QS3",
  "gene_symbol": "ARX"
}